positive regulation of erythrocyte differentiation [GO:0045648] (biological process) Definition: Any process that activates or increases the frequency, rate or extent of erythrocyte differentiation. Sources: GOC:go_curators Also known as: positive regulation of RBC differentiation, positive regulation of red blood cell differentiation, up regulation of erythrocyte differentiation, up-regulation of erythrocyte differentiation, upregulation of erythrocyte differentiation, activation of erythrocyte differentiation, stimulation of erythrocyte differentiation Relationships: is_a positive regulation of myeloid cell differentiation [GO:0045639]; is a type of regulation of erythrocyte differentiation [GO:0045646]; positively regulates GO:0030218